{
  "term_label": "Unknown biological process",
  "gene_symbol": "KLHDC2",
  "term_id": "UNKNOWN:0002",
  "gene": "UniProtKB:Q9Y2U9",
  "gene_name": "Kelch domain-containing protein 2"
}